{
  "gene_name": "Amine oxidase [flavin-containing] A",
  "term_id": "GO:0008131",
  "term_label": "primary methylamine oxidase activity",
  "gene": "UniProtKB:P21397",
  "gene_symbol": "MAOA"
}